{
  "term_label": "SREBP signaling pathway",
  "gene_name": "Rho guanine nucleotide exchange factor 10-like protein",
  "gene_symbol": "ARHGEF10L",
  "term_id": "GO:0032933",
  "gene": "UniProtKB:Q9HCE6"
}